{
  "term_label": "integrin-mediated signaling pathway",
  "gene_symbol": "ITGA4",
  "gene": "UniProtKB:P13612",
  "term_id": "GO:0007229",
  "gene_name": "Integrin alpha-4"
}